{
  "gene_name": "Proline-rich protein 7",
  "gene": "UniProtKB:Q8TB68",
  "term_id": "GO:0099092",
  "gene_symbol": "PRR7",
  "term_label": "postsynaptic density, intracellular component"
}